{
  "gene_symbol": "PPP4R4",
  "gene_name": "Serine_threonine-protein phosphatase 4 regulatory subunit 4",
  "gene": "UniProtKB:Q6NUP7",
  "term_label": "protein serine/threonine phosphatase complex",
  "term_id": "GO:0008287"
}